sphingolipid biosynthesis involved in endoplasmic reticulum membrane organization [GO:0090159] (biological process) Definition: The chemical reactions and pathways resulting in the formation of sphingolipids that contributes to endoplasmic reticulum membrane organization. Relationships: is a type of sphingolipid biosynthetic process [GO:0030148]; is part of GO:0090158 Sources: GOC:ascb_2009, GOC:dph, GOC:tb Also known as: sphingolipid biosynthesis involved in endoplasmic reticulum membrane organisation